{
  "gene": "UniProtKB:Q99829",
  "gene_name": "Copine-1",
  "gene_symbol": "CPNE1",
  "term_label": "plasma membrane",
  "term_id": "GO:0005886"
}